{
  "gene_symbol": "CHRNB2",
  "term_id": "GO:0051899",
  "gene_name": "Neuronal acetylcholine receptor subunit beta-2",
  "term_label": "membrane depolarization",
  "gene": "UniProtKB:P17787"
}